{
  "gene_name": "Ethanolamine kinase 1",
  "term_label": "ethanolamine kinase activity",
  "term_id": "GO:0004305",
  "gene": "UniProtKB:Q9HBU6",
  "gene_symbol": "ETNK1"
}